regulation of antigen processing and presentation via MHC class Ib [GO:0002592] (BP) Sources: GOC:add Subtypes: GO:0002593, positive regulation of antigen processing and presentation via MHC class Ib [GO:0002594], regulation of antigen processing and presentation of peptide antigen via MHC class Ib [GO:0002595], regulation of antigen processing and presentation of lipid antigen via MHC class Ib [GO:0002598] Definition: Any process that modulates the frequency, rate, or extent of antigen processing and presentation of antigen via MHC class Ib. Relationships: is a type of regulation of antigen processing and presentation [GO:0002577]; regulates antigen processing and presentation via MHC class Ib [GO:0002475]